{
  "term_id": "GO:0045177",
  "gene": "UniProtKB:O75970",
  "term_label": "apical part of cell",
  "gene_symbol": "MPDZ",
  "gene_name": "Multiple PDZ domain protein"
}